{
  "gene_name": "Phosphorylase b kinase regulatory subunit alpha, liver isoform",
  "gene_symbol": "PHKA2",
  "term_label": "Unknown biological process",
  "term_id": "UNKNOWN:0002",
  "gene": "UniProtKB:P46019"
}